{
  "term_id": "GO:0090090",
  "term_label": "negative regulation of canonical Wnt signaling pathway",
  "gene_symbol": "DACT3",
  "gene_name": "Dapper homolog 3",
  "gene": "UniProtKB:Q96B18"
}